HLA-B specific inhibitory MHC class I receptor activity [GO:0030109] (molecular function) Definition: Combining with a MHC class I molecule of the HLA-B subclass to mediate signaling that inhibits activation of a lymphocyte. Relationships: is a type of inhibitory MHC class I receptor activity [GO:0032396] References: PMID:11929129, PMID:9368779 Sources: GOC:add, GOC:mah